positive regulation of B cell tolerance induction [GO:0002663] (biological process) Also known as: positive regulation of B lymphocyte tolerance induction, positive regulation of B-cell tolerance induction, positive regulation of B-lymphocyte tolerance induction, up regulation of B cell tolerance induction, up-regulation of B cell tolerance induction, upregulation of B cell tolerance induction, activation of B cell tolerance induction, stimulation of B cell tolerance induction Sources: GOC:add Definition: Any process that activates or increases the frequency, rate, or extent of B cell tolerance induction. Relationships: is_a positive regulation of tolerance induction [GO:0002645]; is a type of GO:0002661; positively regulates GO:0002514 Subtypes: positive regulation of B cell anergy [GO:0002672], positive regulation of B cell deletion [GO:0002869], positive regulation of central B cell tolerance induction [GO:0002897]